{
  "gene": "UniProtKB:P78559",
  "gene_name": "Microtubule-associated protein 1A",
  "term_id": "GO:0031114",
  "gene_symbol": "MAP1A",
  "term_label": "regulation of microtubule depolymerization"
}